tuft [GO:0151001] (cellular component) References: PMID:15817800, PMID:35237268 Definition: A dense cluster of elongated, thick microvilli on the apical surface of tuft cells in epithelial tissues, such as the intestine and respiratory tract. The apical tuft extends further into the lumen than typical microvilli, featuring larger, more compact projections with unique actin cores that penetrate deep into the cytoplasm, often reaching the perinuclear region. This distinctive structure, rich in microfilaments and microtubules, supports the chemosensory functions of the cell. Relationships: is a type of GO:0098862; has part GO:0005902